peptidyl-aspartic acid autophosphorylation [GO:1990938] (biological process) References: PMID:26134396 Sources: GOC:PARL, GOC:bf Relationships: is a type of peptidyl-aspartic acid phosphorylation [GO:0018217]; is_a GO:0046777 Also known as: aspartyl autophosphorylation, peptidyl-aspartate autophosphorylation Definition: The phosphorylation by a protein of one or more of its own aspartate amino acid residues, or an aspartate residue on an identical protein.